creatine:sodium symporter activity [GO:0005309] (molecular function) Relationships: is a type of creatine transmembrane transporter activity [GO:0005308]; is a type of organic acid:sodium symporter activity [GO:0005343] Definition: Enables the transfer of a solute or solutes from one side of a membrane to the other according to the reaction: creatine(out) + Na+(out) = creatine(in) + Na+(in). Sources: TC:2.A.22.3.4 Also known as: sodium/chloride-dependent creatine transporter